{
  "gene_symbol": "ITGB7",
  "gene": "UniProtKB:P26010",
  "gene_name": "Integrin beta-7",
  "term_id": "GO:0009986",
  "term_label": "cell surface"
}